{
  "term_id": "GO:0032587",
  "gene": "UniProtKB:Q9BQI7",
  "gene_name": "PH and SEC7 domain-containing protein 2",
  "term_label": "ruffle membrane",
  "gene_symbol": "PSD2"
}